{
  "term_id": "UNKNOWN:0003",
  "gene_symbol": "PCOTH",
  "gene_name": "Prostate collagen triple helix protein",
  "term_label": "Unknown cellular component",
  "gene": "UniProtKB:Q58A44"
}